{
  "term_id": "GO:0030010",
  "gene_name": "Leucine repeat adapter protein 25",
  "gene": "UniProtKB:Q8N5H3",
  "term_label": "establishment of cell polarity",
  "gene_symbol": "FAM89B"
}